endothelial stalk cell fate specification [GO:0097103] (biological process) Definition: The process involved in the specification of identity of an endothelial stalk cell. Once specification has taken place, a cell will be committed to differentiate down a specific pathway if left in its normal environment. An endothelial stalk cell is a specialized endothelial cell which follows behind the tip cell of an angiogenic sprout. References: PMID:21521739 Sources: CL:0002671, GOC:dgh Relationships: is a type of blood vessel endothelial cell fate specification [GO:0097101]; is part of sprouting angiogenesis [GO:0002040] Also known as: angiogenic stalk cell fate specification